{
  "gene": "UniProtKB:Q9Y4P9",
  "gene_symbol": "SPEF1",
  "gene_name": "Sperm flagellar protein 1",
  "term_label": "axoneme",
  "term_id": "GO:0005930"
}